regulation of IRE1-mediated unfolded protein response [GO:1903894] (biological process) References: PMID:22013210 Sources: GOC:PARL, GOC:TermGenie, GOC:bf, GO_REF:0000058 Also known as: regulation of IRE1 signal transduction pathway, regulation of IRE1 branch of UPR, regulation of UPR signaling by IRE1 stress sensor, regulation of endoplasmic reticulum unfolded protein response; IRE1 signaling, regulation of IRE1alpha unfolded protein response, regulation of IRE1p unfolded protein response, regulation of ERN1-mediated unfolded protein response, regulation of IRE1 signaling in response to endoplasmic reticulum stress, regulation of inositol-requiring transmembrane kinase/endonuclease signal transduction Relationships: is a type of regulation of endoplasmic reticulum unfolded protein response [GO:1900101]; regulates IRE1-mediated unfolded protein response [GO:0036498] Subtypes: GO:1903895, GO:1903896 Definition: Any process that modulates the frequency, rate or extent of the IRE1-mediated unfolded protein response.